{
  "gene_name": "SAM and SH3 domain-containing protein 3",
  "term_id": "GO:0002639",
  "term_label": "positive regulation of immunoglobulin production",
  "gene_symbol": "SASH3",
  "gene": "UniProtKB:O75995"
}